tRNA (adenine-N6)-methyltransferase activity [GO:0016430] (molecular function) Definition: Catalysis of the reaction: S-adenosyl-L-methionine + tRNA = S-adenosyl-L-homocysteine + tRNA containing N6-methyladenine. Sources: EC:2.1.1.55 Also known as: tRNA (adenine-N6-)-methyltransferase activity, S-adenosyl-L-methionine:tRNA (adenine-6-N-)-methyltransferase activity, S-adenosyl-L-methionine:tRNA (adenine-N6-)-methyltransferase activity Relationships: is a type of N-methyltransferase activity [GO:0008170]; is a type of tRNA (adenine) methyltransferase activity [GO:0016426]